negative regulation of mesonephric glomerular mesangial cell proliferation [GO:2000091] (BP) Relationships: is a type of negative regulation of glomerular mesangial cell proliferation [GO:0072125]; is a type of regulation of mesonephric glomerular mesangial cell proliferation [GO:2000090]; is_a negative regulation of cell proliferation involved in mesonephros development [GO:2000607]; negatively regulates mesonephric glomerular mesangial cell proliferation involved in mesonephros development [GO:0061269] Definition: Any process that stops, prevents, or reduces the frequency, rate or extent of mesonephric glomerular mesangial cell proliferation. Sources: GOC:mtg_kidney_jan10